{
  "term_id": "UNKNOWN:0001",
  "term_label": "Unknown molecular function",
  "gene_symbol": "CCDC9",
  "gene_name": "Coiled-coil domain-containing protein 9",
  "gene": "UniProtKB:Q9Y3X0"
}